alanine biosynthetic process [GO:0006523] (biological process) Also known as: alanine anabolism, alanine biosynthesis, alanine formation, alanine synthesis Definition: The chemical reactions and pathways resulting in the formation of alanine, 2-aminopropanoic acid. Sources: GOC:go_curators Subtypes: GO:0030632, L-alanine biosynthetic process [GO:0042852] Relationships: is a type of alanine metabolic process [GO:0006522]; is a type of alpha-amino acid biosynthetic process [GO:1901607]